{
  "term_label": "mediator complex",
  "gene_symbol": "MED8",
  "gene_name": "Mediator of RNA polymerase II transcription subunit 8",
  "term_id": "GO:0016592",
  "gene": "UniProtKB:Q96G25"
}